negative regulation of metanephric ureteric bud development [GO:2001075] (biological process) Sources: GOC:obol Relationships: is a type of negative regulation of developmental process [GO:0051093]; is_a regulation of metanephric ureteric bud development [GO:2001074]; negatively regulates GO:0035502 Definition: Any process that stops, prevents or reduces the frequency, rate or extent of metanephric ureteric bud development.